{
  "gene_name": "Charged multivesicular body protein 6",
  "term_label": "vesicle budding from membrane",
  "gene_symbol": "CHMP6",
  "gene": "UniProtKB:Q96FZ7",
  "term_id": "GO:0006900"
}